{
  "term_label": "regulation of transcription by RNA polymerase II",
  "gene": "UniProtKB:Q8WYN3",
  "term_id": "GO:0006357",
  "gene_symbol": "CSRNP3",
  "gene_name": "Cysteine_serine-rich nuclear protein 3"
}